zymosterol metabolic process [GO:0036196] (biological process) Sources: GOC:yaf Relationships: is a type of sterol metabolic process [GO:0016125]; is_a secondary alcohol metabolic process [GO:1902652] Definition: The chemical reactions and pathways involving zymosterol, (5alpha-cholesta-8,24-dien-3beta-ol). Subtypes: zymosterol biosynthetic process [GO:0036197]